{
  "gene_symbol": "IGHG4",
  "term_label": "immunoglobulin complex, circulating",
  "gene": "UniProtKB:P01861",
  "term_id": "GO:0042571",
  "gene_name": "Immunoglobulin heavy constant gamma 4"
}